{
  "term_label": "chromatin binding",
  "gene": "UniProtKB:Q92794",
  "gene_name": "Histone acetyltransferase KAT6A",
  "term_id": "GO:0003682",
  "gene_symbol": "KAT6A"
}